{
  "term_label": "single-stranded DNA binding",
  "gene_symbol": "ERCC5",
  "gene_name": "DNA excision repair protein ERCC-5",
  "term_id": "GO:0003697",
  "gene": "UniProtKB:P28715"
}